cholesterol metabolic process [GO:0008203] (biological process) Also known as: cholesterol metabolism Definition: The chemical reactions and pathways involving cholesterol, cholest-5-en-3 beta-ol, the principal sterol of vertebrates and the precursor of many steroids, including bile acids and steroid hormones. It is a component of the plasma membrane lipid bilayer and of plasma lipoproteins and can be found in all animal tissues. Regulation: regulated by GO:0090181; positively regulated by positive regulation of cholesterol metabolic process [GO:0090205]; negatively regulated by GO:0090206 Relationships: is a type of GO:0016125; is a type of secondary alcohol metabolic process [GO:1902652] Sources: ISBN:0198506732 Subtypes: GO:0006695, cholesterol catabolic process [GO:0006707], cholesterol ester hydrolysis involved in cholesterol transport [GO:0090122]